{
  "gene_symbol": "G2E3",
  "gene_name": "G2_M phase-specific E3 ubiquitin-protein ligase",
  "gene": "UniProtKB:Q7L622",
  "term_label": "Unknown molecular function",
  "term_id": "UNKNOWN:0001"
}